regulation of branching involved in salivary gland morphogenesis [GO:0060693] (biological process) Relationships: is a type of GO:0060688; is a type of regulation of morphogenesis of an epithelium [GO:1905330]; is a type of GO:2000027; regulates branching involved in salivary gland morphogenesis [GO:0060445] Definition: Any process that modulates the rate, frequency, or extent of branching morphogenesis in the salivary gland epithelium. Subtypes: GO:0060665, regulation of branching involved in salivary gland morphogenesis by extracellular matrix-epithelial cell signaling [GO:0060668], regulation of branching involved in salivary gland morphogenesis by epithelial-mesenchymal signaling [GO:0060683] Sources: GOC:dph